{
  "gene_symbol": "PSMC3IP",
  "gene_name": "Homologous-pairing protein 2 homolog",
  "gene": "UniProtKB:Q9P2W1",
  "term_label": "homologous chromosome pairing at meiosis",
  "term_id": "GO:0007129"
}